{
  "term_id": "GO:0032528",
  "gene": "UniProtKB:O43490",
  "gene_name": "Prominin-1",
  "gene_symbol": "PROM1",
  "term_label": "microvillus organization"
}